{
  "gene": "UniProtKB:Q16635",
  "term_id": "GO:0031966",
  "gene_name": "Tafazzin",
  "term_label": "mitochondrial membrane",
  "gene_symbol": "TAFAZZIN"
}